cellular response to alkane [GO:1902779] (biological process) Subtypes: cellular response to nonane [GO:1902781], cellular response to decane [GO:1902783], cellular response to undecane [GO:1902785], cellular response to dodecane [GO:1902787], cellular response to isooctane [GO:1902789] Definition: Any process that results in a change in state or activity of a cell (in terms of movement, secretion, enzyme production, gene expression, etc.) as a result of an alkane stimulus. References: PMID:22958739, PMID:23826995 Sources: GOC:TermGenie, GOC:mengo_curators, GO_REF:0000071 Relationships: is a type of cellular response to chemical stimulus [GO:0070887]; is a type of response to alkane [GO:1902778]